{
  "gene_symbol": "MON2",
  "gene_name": "Protein MON2 homolog",
  "term_id": "GO:0042147",
  "gene": "UniProtKB:Q7Z3U7",
  "term_label": "retrograde transport, endosome to Golgi"
}